{
  "gene_name": "Keratin-associated protein 1-1",
  "term_id": "UNKNOWN:0002",
  "gene": "UniProtKB:Q07627",
  "term_label": "Unknown biological process",
  "gene_symbol": "KRTAP1-1"
}